{
  "term_id": "GO:0051058",
  "gene_symbol": "GMIP",
  "gene": "UniProtKB:Q9P107",
  "gene_name": "GEM-interacting protein",
  "term_label": "negative regulation of small GTPase mediated signal transduction"
}